{
  "term_id": "UNKNOWN:0002",
  "gene_symbol": "WDR31",
  "gene_name": "WD repeat-containing protein 31",
  "gene": "UniProtKB:Q8NA23",
  "term_label": "Unknown biological process"
}